{
  "gene_name": "V(D)J recombination-activating protein 1",
  "gene": "UniProtKB:P15918",
  "gene_symbol": "RAG1",
  "term_id": "GO:0002250",
  "term_label": "adaptive immune response"
}